embryonic cranial skeleton morphogenesis [GO:0048701] (BP) Relationships: is a type of embryonic skeletal system morphogenesis [GO:0048704]; is part of cranial skeletal system development [GO:1904888] References: PMID:16049113 Sources: GOC:dsf, GOC:jid Definition: The process in which the anatomical structures of the cranial skeleton are generated and organized during the embryonic phase. Also known as: embryonic cranium morphogenesis